regulation of isopentenyl diphosphate biosynthetic process, methylerythritol 4-phosphate pathway [GO:0010322] (biological process) Relationships: is a type of regulation of carbohydrate metabolic process [GO:0006109]; is a type of regulation of ketone metabolic process [GO:0010565]; is_a GO:0019747; is a type of regulation of phospholipid biosynthetic process [GO:0071071]; regulates isopentenyl diphosphate biosynthetic process, methylerythritol 4-phosphate pathway [GO:0019288] References: PMID:16531478 Subtypes: negative regulation of isopentenyl diphosphate biosynthetic process, methylerythritol 4-phosphate pathway [GO:0010323] Also known as: regulation of isopentenyl diphosphate biosynthetic process, mevalonate-independent pathway Definition: Any process that modulates the frequency, rate or extent of the chemical reactions and pathways resulting in the formation of isopentenyl diphosphate produced via the methylerythritol (MEP) pathway (mevalonate-independent).